{
  "term_id": "UNKNOWN:0002",
  "gene_name": "tRNA (adenine(37)-N6)-methyltransferase",
  "gene_symbol": "TRMO",
  "gene": "UniProtKB:Q9BU70",
  "term_label": "Unknown biological process"
}